{
  "term_id": "GO:0000149",
  "gene_symbol": "EXOC3",
  "term_label": "SNARE binding",
  "gene": "UniProtKB:O60645",
  "gene_name": "Exocyst complex component 3"
}